{
  "gene": "UniProtKB:Q01628",
  "term_label": "response to interferon-beta",
  "gene_symbol": "IFITM3",
  "gene_name": "Interferon-induced transmembrane protein 3",
  "term_id": "GO:0035456"
}